5-methyltetrahydropteroyltriglutamate-homocysteine S-methyltransferase activity [GO:0003871] (molecular function) Relationships: is a type of GO:0008172; is a type of 5-methyltetrahydropteroyltri-L-glutamate-dependent methyltransferase activity [GO:0042085] Definition: Catalysis of the reaction: 5-methyltetrahydropteroyltri-L-glutamate + L-homocysteine = L-methionine + tetrahydropteroyltri-L-glutamate. Sources: EC:2.1.1.14, RHEA:21196 Also known as: 5-methyltetrahydropteroyltri-L-glutamate:L-homocysteine S-methyltransferase activity, MetE, cobalamin-independent methionine synthase activity, homocysteine methylase activity, methionine synthase (cobalamin-independent) activity, methyltetrahydropteroylpolyglutamate:homocysteine methyltransferase activity, methyltransferase, tetrahydropteroylglutamate-homocysteine transmethylase activity, tetrahydropteroylglutamate-homocysteine transmethylase activity, tetrahydropteroyltriglutamate methyltransferase activity